{
  "term_label": "protein localization to plasma membrane",
  "gene": "UniProtKB:P41743",
  "gene_symbol": "PRKCI",
  "gene_name": "Protein kinase C iota type",
  "term_id": "GO:0072659"
}